{
  "term_id": "GO:0005783",
  "gene": "UniProtKB:Q8NBS9",
  "gene_symbol": "TXNDC5",
  "term_label": "endoplasmic reticulum",
  "gene_name": "Thioredoxin domain-containing protein 5"
}